{
  "term_label": "serine-type endopeptidase activity",
  "gene_symbol": "UBAC2",
  "term_id": "GO:0004252",
  "gene_name": "Ubiquitin-associated domain-containing protein 2",
  "gene": "UniProtKB:Q8NBM4"
}